prenylation [GO:0097354] (biological process) Subtypes: protein prenylation [GO:0018342] References: PMID:18029206, PMID:21351751, PMID:22123822, PMID:22642693, PMID:22660767 Sources: GOC:di Relationships: is a type of metabolic process [GO:0008152] Definition: The covalent attachment of a prenyl group to a molecule; geranyl, farnesyl, or geranylgeranyl groups may be added.